{
  "gene": "UniProtKB:Q9H8G1",
  "gene_symbol": "ZNF430",
  "term_id": "GO:0000978",
  "gene_name": "Zinc finger protein 430",
  "term_label": "RNA polymerase II cis-regulatory region sequence-specific DNA binding"
}